{
  "term_id": "UNKNOWN:0003",
  "gene_symbol": "TCEAL7",
  "gene_name": "Transcription elongation factor A protein-like 7",
  "term_label": "Unknown cellular component",
  "gene": "UniProtKB:Q9BRU2"
}